{
  "term_id": "GO:0000981",
  "gene": "UniProtKB:P50553",
  "gene_symbol": "ASCL1",
  "gene_name": "Achaete-scute homolog 1",
  "term_label": "DNA-binding transcription factor activity, RNA polymerase II-specific"
}